{
  "gene": "UniProtKB:A0A1B0GTU1",
  "gene_name": "Zinc finger CCCH domain-containing protein 11B",
  "gene_symbol": "ZC3H11B",
  "term_id": "GO:0003729",
  "term_label": "mRNA binding"
}